{
  "term_label": "histone H3K9 demethylase activity",
  "gene": "UniProtKB:Q6B0I6",
  "gene_name": "Lysine-specific demethylase 4D",
  "term_id": "GO:0032454",
  "gene_symbol": "KDM4D"
}